{
  "term_label": "GET complex",
  "gene": "UniProtKB:P49069",
  "gene_symbol": "CAMLG",
  "gene_name": "Guided entry of tail-anchored proteins factor CAMLG",
  "term_id": "GO:0043529"
}